neuropeptide receptor binding [GO:0071855] (molecular function) Subtypes: apelin receptor binding [GO:0031704], GO:0031705, cholecystokinin receptor binding [GO:0031739], galanin receptor binding [GO:0031763], GO:0031770, GO:0031773, melanin-concentrating hormone receptor binding [GO:0031776], melanocortin receptor binding [GO:0031779], neurokinin receptor binding [GO:0031834], neuropeptide Y receptor binding [GO:0031841], neurotensin receptor binding [GO:0031846], GO:0031854, pituitary adenylate cyclase-activating polypeptide receptor binding [GO:0031858], prolactin-releasing peptide receptor binding [GO:0031861], somatostatin receptor binding [GO:0031877], vasoactive intestinal polypeptide receptor binding [GO:0031890], orexin receptor binding [GO:0042324], neuromedin U receptor binding [GO:0042922], corticotropin-releasing hormone receptor binding [GO:0051429], beta-endorphin receptor binding [GO:0071857], corazonin receptor binding [GO:0071858], neuropeptide F receptor binding [GO:0071859], proctolin receptor binding [GO:0071860], tachykinin receptor binding [GO:0071861] Sources: GOC:kmv, GOC:mah Definition: Binding to a neuropeptide receptor. Relationships: is a type of G protein-coupled receptor binding [GO:0001664]